cytosol to endoplasmic reticulum transport [GO:0046967] (biological process) Relationships: is a type of GO:0046907; is a type of transmembrane transport [GO:0055085] Subtypes: GDP-fucose import into endoplasmic reticulum lumen [GO:0036084], UDP-glucose transmembrane transport into endoplasmic reticulum [GO:0120112], GO:0140209, magnesium ion transport from cytosol to endoplasmic reticulum [GO:0160176], calcium ion transport from cytosol to endoplasmic reticulum [GO:1903515] Sources: GOC:ai Definition: The directed movement of substances from the cytosol to the endoplasmic reticulum of a cell. Also known as: cytosol to ER transport